{
  "gene_symbol": "MKRN9P",
  "term_label": "Unknown cellular component",
  "gene": "UniProtKB:Q6NVV0",
  "term_id": "UNKNOWN:0003",
  "gene_name": "Putative makorin-5"
}